endolysosome membrane [GO:0036020] (cellular component) Sources: GOC:pde Also known as: endolysosomal membrane Definition: The lipid bilayer surrounding an endolysosome. An endolysosome is a transient hybrid organelle formed by fusion of a late endosome with a lysosome. Relationships: is a type of GO:0005765; is a type of GO:0010008; is part of endolysosome [GO:0036019]